{
  "gene": "UniProtKB:Q9NZQ0",
  "gene_symbol": "DNAJC27",
  "term_id": "GO:0006886",
  "term_label": "intracellular protein transport",
  "gene_name": "DnaJ homolog subfamily C member 27"
}